solitary nucleus development [GO:0021746] (biological process) Definition: The process whose specific outcome is the progression of the solitary nucleus over time, from its formation to the mature structure. Relationships: is a type of neural nucleus development [GO:0048857]; is part of medulla oblongata development [GO:0021550] Sources: GOC:cls, GOC:curators, GOC:dgh, GOC:dph, GOC:jid